{
  "gene": "UniProtKB:P48645",
  "gene_symbol": "NMU",
  "term_id": "GO:0042922",
  "term_label": "neuromedin U receptor binding",
  "gene_name": "Neuromedin-U"
}